{
  "gene_symbol": "MMP24",
  "term_label": "metalloendopeptidase activity",
  "gene": "UniProtKB:Q9Y5R2",
  "gene_name": "Matrix metalloproteinase-24",
  "term_id": "GO:0004222"
}